positive regulation of RIG-I signaling pathway [GO:1900246] (biological process) Definition: Any process that activates or increases the frequency, rate or extent of RIG-I signaling pathway. Relationships: is a type of regulation of RIG-I signaling pathway [GO:0039535]; is a type of positive regulation of pattern recognition receptor signaling pathway [GO:0062208]; is a type of GO:1902533; positively regulates GO:0039529 Also known as: positive regulation of DDX58 signaling pathway, positive regulation of RIG-I signalling pathway, positive regulation of retinoic acid inducible gene I signaling pathway, up regulation of DDX58 signaling pathway, up regulation of RIG-I signaling pathway, up regulation of retinoic acid inducible gene I signaling pathway, up-regulation of DDX58 signaling pathway, up-regulation of RIG-I signaling pathway, up-regulation of retinoic acid inducible gene I signaling pathway, upregulation of DDX58 signaling pathway, upregulation of RIG-I signaling pathway, upregulation of retinoic acid inducible gene I signaling pathway, activation of DDX58 signaling pathway, activation of RIG-I signaling pathway, activation of retinoic acid inducible gene I signaling pathway Sources: GOC:TermGenie